{
  "gene": "UniProtKB:Q5TA31",
  "gene_name": "E3 ubiquitin-protein ligase RNF187",
  "term_label": "Unknown cellular component",
  "gene_symbol": "RNF187",
  "term_id": "UNKNOWN:0003"
}